{
  "term_label": "Unknown biological process",
  "term_id": "UNKNOWN:0002",
  "gene_name": "UPF0545 protein C22orf39",
  "gene_symbol": "C22orf39",
  "gene": "UniProtKB:Q6P5X5"
}